{
  "term_label": "positive regulation of Rho protein signal transduction",
  "gene": "UniProtKB:Q12802",
  "term_id": "GO:0035025",
  "gene_name": "A-kinase anchor protein 13",
  "gene_symbol": "AKAP13"
}